calcium-dependent self proteolysis [GO:1990092] (biological process) Definition: The calcium-dependent hydrolysis of proteins into smaller polypeptides and/or amino acids by cleavage of their own peptide bonds. References: PMID:20460380 Relationships: is a type of self proteolysis [GO:0097264]